{
  "term_label": "maturation of 5.8S rRNA",
  "term_id": "GO:0000460",
  "gene": "UniProtKB:Q9Y3B9",
  "gene_symbol": "RRP15",
  "gene_name": "RRP15-like protein"
}